interleukin-8 binding [GO:0019959] (molecular function) Also known as: IL-8 binding Sources: GOC:jl Definition: Binding to interleukin-8. Relationships: is a type of C-X-C chemokine binding [GO:0019958]